regulation of fat cell apoptotic process [GO:1904649] (biological process) References: PMID:17024416 Sources: GOC:TermGenie, GO_REF:0000058 Subtypes: negative regulation of fat cell apoptotic process [GO:1904650], GO:1904651 Relationships: is a type of GO:0042981; RO_0002211 fat cell apoptotic process [GO:1904606] Definition: Any process that modulates the frequency, rate or extent of fat cell apoptotic process. Also known as: regulation of adipocyte apoptotic process, regulation of adipose cell apoptotic process, regulation of adipocyte apoptosis, regulation of adipose cell apoptosis, regulation of fat cell apoptosis